{
  "gene_name": "Guanosine-3',5'-bis(diphosphate) 3'-pyrophosphohydrolase MESH1",
  "term_label": "Unknown cellular component",
  "gene": "UniProtKB:Q8N4P3",
  "gene_symbol": "HDDC3",
  "term_id": "UNKNOWN:0003"
}